{
  "gene_symbol": "ZNF571",
  "term_label": "DNA-binding transcription factor activity, RNA polymerase II-specific",
  "gene_name": "Zinc finger protein 571",
  "gene": "UniProtKB:Q7Z3V5",
  "term_id": "GO:0000981"
}